{
  "term_id": "GO:0070602",
  "term_label": "regulation of centromeric sister chromatid cohesion",
  "gene": "UniProtKB:Q9Y2T1",
  "gene_symbol": "AXIN2",
  "gene_name": "Axin-2"
}